smooth muscle cell differentiation [GO:0051145] (BP) Subtypes: enteric smooth muscle cell differentiation [GO:0035645], GO:0035886, smooth muscle cell differentiation involved in prostate glandular acinus development [GO:0060530], GO:0072193, kidney smooth muscle cell differentiation [GO:0072195] Regulation: regulated by regulation of smooth muscle cell differentiation [GO:0051150]; negatively regulated by negative regulation of smooth muscle cell differentiation [GO:0051151]; positively regulated by GO:0051152 Relationships: is a type of muscle cell differentiation [GO:0042692] Sources: CL:0000192, GOC:ai Also known as: nonstriated muscle cell differentiation Definition: The process in which a relatively unspecialized cell acquires specialized features of a smooth muscle cell; smooth muscle lacks transverse striations in its constituent fibers and are almost always involuntary.